{
  "gene_symbol": "UBE4A",
  "term_label": "protein polyubiquitination",
  "gene": "UniProtKB:Q14139",
  "term_id": "GO:0000209",
  "gene_name": "Ubiquitin conjugation factor E4 A"
}